regulation of exocytosis [GO:0017157] (biological process) Relationships: is a type of regulation of vesicle-mediated transport [GO:0060627]; is a type of regulation of secretion by cell [GO:1903530]; regulates exocytosis [GO:0006887] Definition: Any process that modulates the frequency, rate or extent of exocytosis. Sources: GOC:go_curators Subtypes: negative regulation of exocytosis [GO:0045920], positive regulation of exocytosis [GO:0045921], regulation of exocytic insertion of neurotransmitter receptor to postsynaptic membrane [GO:0099145], regulation of regulated secretory pathway [GO:1903305], regulation of constitutive secretory pathway [GO:1903433], regulation of exosomal secretion [GO:1903541]